positive regulation of phosphorus utilization [GO:0045949] (biological process) Definition: Any process that activates or increases the frequency, rate or extent of phosphorus utilization. Sources: GOC:go_curators Also known as: up regulation of phosphorus utilization, up-regulation of phosphorus utilization, upregulation of phosphorus utilization, activation of phosphorus utilization, stimulation of phosphorus utilization Relationships: is a type of regulation of phosphorus utilization [GO:0006795]; is a type of positive regulation of phosphorus metabolic process [GO:0010562]; positively regulates phosphorus utilization [GO:0006794]